{
  "gene_name": "SUN domain-containing protein 2",
  "term_id": "GO:0034993",
  "gene_symbol": "SUN2",
  "term_label": "meiotic nuclear membrane microtubule tethering complex",
  "gene": "UniProtKB:Q9UH99"
}